{
  "term_label": "nucleus",
  "term_id": "GO:0005634",
  "gene_symbol": "SRPK2",
  "gene_name": "SRSF protein kinase 2",
  "gene": "UniProtKB:P78362"
}